{
  "term_label": "mitochondrial outer membrane",
  "gene_name": "Mitofusin-1",
  "gene": "UniProtKB:Q8IWA4",
  "gene_symbol": "MFN1",
  "term_id": "GO:0005741"
}